{
  "term_label": "pentose metabolic process",
  "term_id": "GO:0019321",
  "gene_name": "FGGY carbohydrate kinase domain-containing protein",
  "gene": "UniProtKB:Q96C11",
  "gene_symbol": "FGGY"
}